{
  "term_label": "EMC complex",
  "term_id": "GO:0072546",
  "gene": "UniProtKB:Q9NPA0",
  "gene_symbol": "EMC7",
  "gene_name": "ER membrane protein complex subunit 7"
}